{
  "term_label": "positive regulation of transcription by RNA polymerase II",
  "gene": "UniProtKB:Q76L83",
  "gene_symbol": "ASXL2",
  "term_id": "GO:0045944",
  "gene_name": "Putative Polycomb group protein ASXL2"
}